trehalose 6-phosphate phosphorylase activity [GO:0050503] (MF) Definition: Catalysis of the reaction: trehalose 6-phosphate + phosphate = glucose 6-phosphate + beta-D-glucose 1-phosphate. Relationships: is a type of 1,4-alpha-oligoglucan phosphorylase activity [GO:0004645] Also known as: trehalose 6-phosphate:phosphate beta-D-glucosyltransferase activity Sources: EC:2.4.1.216, MetaCyc:2.4.1.216-RXN